{
  "term_label": "regulation of cytosolic calcium ion concentration",
  "gene_symbol": "CALCA",
  "gene": "UniProtKB:P01258",
  "term_id": "GO:0051480",
  "gene_name": "Calcitonin"
}